protein localization to microtubule minus-end [GO:1904519] (biological process) References: PMID:25987607 Sources: GOC:TermGenie, GO_REF:0000087 Relationships: is a type of protein localization to microtubule end [GO:1905725] Also known as: protein localisation in microtubule minus-end, protein localisation to microtubule minus-end, protein localization in microtubule minus-end Definition: A process in which a protein is transported to, or maintained in, a location at a microtubule minus-end.